{
  "term_label": "CCR chemokine receptor binding",
  "gene_symbol": "CCL5",
  "gene_name": "C-C motif chemokine 5",
  "gene": "UniProtKB:P13501",
  "term_id": "GO:0048020"
}